positive regulation of outer hair cell apoptotic process [GO:1905587] (biological process) Definition: Any process that activates or increases the frequency, rate or extent of outer hair cell apoptotic process. References: PMID:24472721 Sources: GOC:TermGenie, GO_REF:0000058 Also known as: positive regulation of cochlear outer hair cell apoptotic process, up regulation of cochlear outer hair cell apoptotic process, up regulation of outer hair cell apoptotic process, up-regulation of cochlear outer hair cell apoptotic process, up-regulation of outer hair cell apoptotic process, upregulation of cochlear outer hair cell apoptotic process, upregulation of outer hair cell apoptotic process, activation of cochlear outer hair cell apoptosis, activation of cochlear outer hair cell apoptotic process, activation of outer hair cell apoptosis, activation of outer hair cell apoptotic process, positive regulation of cochlear outer hair cell apoptosis, positive regulation of outer hair cell apoptosis, up regulation of cochlear outer hair cell apoptosis, up regulation of outer hair cell apoptosis, up-regulation of cochlear outer hair cell apoptosis, up-regulation of outer hair cell apoptosis, upregulation of cochlear outer hair cell apoptosis, upregulation of outer hair cell apoptosis Relationships: is_a positive regulation of neuron apoptotic process [GO:0043525]; is a type of GO:1905585; positively regulates outer hair cell apoptotic process [GO:1905584]